{
  "gene_symbol": "SSR4",
  "gene": "UniProtKB:P51571",
  "gene_name": "Translocon-associated protein subunit delta",
  "term_id": "UNKNOWN:0002",
  "term_label": "Unknown biological process"
}